{
  "gene_symbol": "ZBTB7C",
  "gene_name": "Zinc finger and BTB domain-containing protein 7C",
  "gene": "UniProtKB:A1YPR0",
  "term_label": "regulation of transcription by RNA polymerase II",
  "term_id": "GO:0006357"
}